{
  "term_id": "GO:0000226",
  "gene": "UniProtKB:Q96EK5",
  "gene_symbol": "KIFBP",
  "gene_name": "KIF-binding protein",
  "term_label": "microtubule cytoskeleton organization"
}